{
  "term_label": "neurogenesis",
  "term_id": "GO:0022008",
  "gene_name": "Diacylglycerol lipase-beta",
  "gene": "UniProtKB:Q8NCG7",
  "gene_symbol": "DAGLB"
}